{
  "gene": "UniProtKB:Q14055",
  "gene_symbol": "COL9A2",
  "term_label": "collagen type IX trimer",
  "term_id": "GO:0005594",
  "gene_name": "Collagen alpha-2(IX) chain"
}